{
  "gene_name": "Alpha-actinin-1",
  "term_label": "muscle cell development",
  "term_id": "GO:0055001",
  "gene_symbol": "ACTN1",
  "gene": "UniProtKB:P12814"
}